muscle myosin complex [GO:0005859] (CC) Sources: GOC:mah Definition: A filament of myosin found in a muscle cell of any type. Relationships: is a type of myosin II complex [GO:0016460]; BFO_0000050 contractile muscle fiber [GO:0043292]